kidney interstitial fibroblast differentiation [GO:0072071] (biological process) Subtypes: mesonephric interstitial fibroblast differentiation [GO:0061266], metanephric interstitial fibroblast differentiation [GO:0072258] Sources: GOC:mtg_kidney_jan10 Also known as: kidney interstitial cell differentiation Definition: The process in which relatively unspecialized cells acquire specialized structural and/or functional features that characterize the interstitial fibroblast of the kidney as it progresses from its formation to the mature state. Relationships: is a type of cell differentiation involved in kidney development [GO:0061005]